{
  "gene_symbol": "H2BC3",
  "gene": "UniProtKB:P33778",
  "term_label": "antimicrobial humoral immune response mediated by antimicrobial peptide",
  "term_id": "GO:0061844",
  "gene_name": "Histone H2B type 1-B"
}